{
  "term_id": "UNKNOWN:0001",
  "gene": "UniProtKB:Q6NYC8",
  "gene_name": "Phostensin",
  "term_label": "Unknown molecular function",
  "gene_symbol": "PPP1R18"
}